{
  "gene_name": "Mediator of RNA polymerase II transcription subunit 18",
  "term_id": "GO:0016592",
  "gene_symbol": "MED18",
  "gene": "UniProtKB:Q9BUE0",
  "term_label": "mediator complex"
}